{
  "term_id": "GO:0005545",
  "gene_symbol": "SNAP91",
  "term_label": "1-phosphatidylinositol binding",
  "gene": "UniProtKB:O60641",
  "gene_name": "Clathrin coat assembly protein AP180"
}